{
  "term_id": "GO:1990817",
  "term_label": "poly(A) RNA polymerase activity",
  "gene": "UniProtKB:P51003",
  "gene_name": "Poly(A) polymerase alpha",
  "gene_symbol": "PAPOLA"
}